{
  "gene_name": "RILP-like protein 1",
  "term_id": "GO:0036064",
  "gene": "UniProtKB:Q5EBL4",
  "term_label": "ciliary basal body",
  "gene_symbol": "RILPL1"
}